{
  "gene_symbol": "KRT10",
  "gene": "UniProtKB:P13645",
  "term_label": "cytoskeleton",
  "gene_name": "Keratin, type I cytoskeletal 10",
  "term_id": "GO:0005856"
}